{
  "gene": "UniProtKB:P04626",
  "gene_symbol": "ERBB2",
  "term_id": "GO:0030182",
  "term_label": "neuron differentiation",
  "gene_name": "Receptor tyrosine-protein kinase erbB-2"
}